{
  "gene": "UniProtKB:Q16665",
  "term_id": "GO:0000977",
  "gene_name": "Hypoxia-inducible factor 1-alpha",
  "term_label": "RNA polymerase II transcription regulatory region sequence-specific DNA binding",
  "gene_symbol": "HIF1A"
}